3M complex [GO:1990393] (cellular component) Definition: A protein complex, at least composed of CUL7, CCDC8 and OBSL1, that is required for maintaining microtubule and genome integrity. Relationships: is a type of protein-containing complex [GO:0032991] References: PMID:24793695, PMID:24793696